{
  "term_label": "TORC2 complex",
  "gene_symbol": "PRR5",
  "gene": "UniProtKB:P85299",
  "term_id": "GO:0031932",
  "gene_name": "Proline-rich protein 5"
}